{
  "term_id": "GO:0030141",
  "term_label": "secretory granule",
  "gene_name": "Ras-related protein Rab-27A",
  "gene_symbol": "RAB27A",
  "gene": "UniProtKB:P51159"
}